{
  "term_id": "GO:0015881",
  "gene_name": "Monocarboxylate transporter 12",
  "term_label": "creatine transmembrane transport",
  "gene": "UniProtKB:Q6ZSM3",
  "gene_symbol": "SLC16A12"
}